{
  "term_id": "GO:0000978",
  "gene_symbol": "ZNF350",
  "term_label": "RNA polymerase II cis-regulatory region sequence-specific DNA binding",
  "gene_name": "Zinc finger protein 350",
  "gene": "UniProtKB:Q9GZX5"
}